{
  "term_id": "UNKNOWN:0002",
  "gene": "UniProtKB:Q9P2E9",
  "gene_name": "Ribosome-binding protein 1",
  "term_label": "Unknown biological process",
  "gene_symbol": "RRBP1"
}